{
  "gene": "UniProtKB:P16112",
  "term_id": "GO:0005615",
  "gene_symbol": "ACAN",
  "term_label": "extracellular space",
  "gene_name": "Aggrecan core protein"
}